{
  "gene_name": "Coiled-coil-helix-coiled-coil-helix domain-containing protein 5",
  "term_label": "Unknown molecular function",
  "term_id": "UNKNOWN:0001",
  "gene_symbol": "CHCHD5",
  "gene": "UniProtKB:Q9BSY4"
}